{
  "gene": "UniProtKB:P01615",
  "gene_symbol": "IGKV2D-28",
  "term_id": "GO:0006955",
  "gene_name": "Immunoglobulin kappa variable 2D-28",
  "term_label": "immune response"
}